{
  "term_label": "cytosol",
  "gene_symbol": "ZFP36",
  "gene_name": "mRNA decay activator protein ZFP36",
  "gene": "UniProtKB:P26651",
  "term_id": "GO:0005829"
}